{
  "gene_name": "Homeobox protein Nkx-2.8",
  "gene": "UniProtKB:O15522",
  "term_id": "GO:0000978",
  "gene_symbol": "NKX2-8",
  "term_label": "RNA polymerase II cis-regulatory region sequence-specific DNA binding"
}